{
  "gene": "UniProtKB:Q9H3T3",
  "gene_symbol": "SEMA6B",
  "gene_name": "Semaphorin-6B",
  "term_id": "GO:0001755",
  "term_label": "neural crest cell migration"
}